regulation of tocopherol cyclase activity [GO:1902171] (biological process) Relationships: is a type of regulation of catalytic activity [GO:0050790]; regulates tocopherol cyclase activity [GO:0009976] References: PMID:23632854 Sources: GOC:TermGenie Definition: Any process that modulates the frequency, rate or extent of tocopherol cyclase activity.